{
  "term_label": "DNA-binding transcription factor activity",
  "gene": "UniProtKB:Q5HYK9",
  "gene_symbol": "ZNF667",
  "gene_name": "Zinc finger protein 667",
  "term_id": "GO:0003700"
}